{
  "gene_symbol": "PDE1C",
  "gene": "UniProtKB:Q14123",
  "term_label": "neuronal cell body",
  "term_id": "GO:0043025",
  "gene_name": "Dual specificity calcium_calmodulin-dependent 3',5'-cyclic nucleotide phosphodiesterase 1C"
}